{
  "gene": "UniProtKB:Q6PIF6",
  "term_label": "sensory perception of sound",
  "gene_name": "Unconventional myosin-VIIb",
  "term_id": "GO:0007605",
  "gene_symbol": "MYO7B"
}